{
  "term_id": "UNKNOWN:0001",
  "gene": "UniProtKB:O75140",
  "term_label": "Unknown molecular function",
  "gene_name": "GATOR complex protein DEPDC5",
  "gene_symbol": "DEPDC5"
}